sodium ion transport [GO:0006814] (biological process) Also known as: sodium/potassium transport, sodium transport, mitochondrial sodium/calcium ion exchange, sodium:calcium exchange, sodium:solute transport, sodium channel auxiliary protein activity Relationships: is a type of metal ion transport [GO:0030001] Sources: GOC:ai Definition: The directed movement of sodium ions (Na+) into, out of or within a cell, or between cells, by means of some agent such as a transporter or pore. Subtypes: renal sodium ion transport [GO:0003096], GO:0035725 Regulation: regulated by GO:0002028; positively regulated by positive regulation of sodium ion transport [GO:0010765]; RO_0002212 by negative regulation of sodium ion transport [GO:0010766]